{
  "gene_symbol": "CWC27",
  "term_label": "catalytic step 2 spliceosome",
  "gene_name": "Spliceosome-associated protein CWC27 homolog",
  "term_id": "GO:0071013",
  "gene": "UniProtKB:Q6UX04"
}